{
  "term_id": "GO:0008630",
  "gene": "UniProtKB:Q07820",
  "gene_symbol": "MCL1",
  "term_label": "intrinsic apoptotic signaling pathway in response to DNA damage",
  "gene_name": "Induced myeloid leukemia cell differentiation protein Mcl-1"
}